cranial nerve structural organization [GO:0021604] (biological process) Sources: GOC:cls, GOC:dgh, GOC:dph, GOC:jid, GO_REF:0000021 Definition: The process that contributes to the act of creating the structural organization of the cranial nerves. This process pertains to the physical shaping of a rudimentary structure. The cranial nerves are composed of twelve pairs of nerves that emanate from the nervous tissue of the hindbrain. These nerves are sensory, motor, or mixed in nature, and provide the motor and general sensory innervation of the head, neck and viscera. They mediate vision, hearing, olfaction and taste and carry the parasympathetic innervation of the autonomic ganglia that control visceral functions. Relationships: is_a anatomical structure arrangement [GO:0048532]; is part of GO:0021602 Also known as: cranial nerve structural organisation Subtypes: abducens nerve structural organization [GO:0021600], accessory nerve structural organization [GO:0021609], facial nerve structural organization [GO:0021612], glossopharyngeal nerve structural organization [GO:0021617], GO:0021621, oculomotor nerve structural organization [GO:0021624], olfactory nerve structural organization [GO:0021629], optic nerve structural organization [GO:0021633], trigeminal nerve structural organization [GO:0021637], trochlear nerve structural organization [GO:0021641], vagus nerve structural organization [GO:0021645], vestibulocochlear nerve structural organization [GO:0021649]